phosphatase inhibitor activity [GO:0019212] (molecular function) Definition: Binds to and stops, prevents or reduces the activity of a phosphatase. Sources: GOC:ai Relationships: is a type of enzyme inhibitor activity [GO:0004857]; is a type of phosphatase regulator activity [GO:0019208]; negatively regulates phosphatase activity [GO:0016791] Subtypes: GO:0001691, protein phosphatase inhibitor activity [GO:0004864]